{
  "gene_name": "Zinc finger protein 34",
  "gene": "UniProtKB:Q8IZ26",
  "term_id": "GO:0000978",
  "gene_symbol": "ZNF34",
  "term_label": "RNA polymerase II cis-regulatory region sequence-specific DNA binding"
}